{
  "gene_name": "Arginyl-tRNA--protein transferase 1",
  "gene": "UniProtKB:O95260",
  "term_label": "arginyl-tRNA--protein transferase activity",
  "gene_symbol": "ATE1",
  "term_id": "GO:0004057"
}